purine ribonucleoside monophosphate metabolic process [GO:0009167] (biological process) Sources: GOC:go_curators, ISBN:0198506732 Definition: The chemical reactions and pathways involving purine ribonucleoside monophosphate, a compound consisting of a purine base linked to a ribose sugar esterified with phosphate on the sugar. Relationships: is a type of purine nucleoside monophosphate metabolic process [GO:0009126] Subtypes: purine ribonucleoside monophosphate biosynthetic process [GO:0009168], purine ribonucleoside monophosphate catabolic process [GO:0009169], AMP metabolic process [GO:0046033], GO:0046037, GO:0046040, XMP metabolic process [GO:0097292] Also known as: purine ribonucleoside monophosphate metabolism